{
  "gene_name": "Coiled-coil domain-containing protein 136",
  "term_label": "acrosome assembly",
  "term_id": "GO:0001675",
  "gene": "UniProtKB:Q96JN2",
  "gene_symbol": "CCDC136"
}